{
  "term_id": "GO:0007417",
  "gene_name": "MARCKS-related protein",
  "gene": "UniProtKB:P49006",
  "term_label": "central nervous system development",
  "gene_symbol": "MARCKSL1"
}